protoperithecium formation [GO:0120166] (biological process) Relationships: is_a GO:0030582 Definition: The process of producing fruiting body precursors, called protoperithecia. Protoperitheicium is a spherical structure that is formed in the sexual phase of ascomycetous fungi such as Neurospora crassa and Sordaria macrospora. Protoperithecium is formed by the enveloping of ascogonia cells by sterile hyphae and it develops into perithecium. References: PMID:125266, PMID:20739093, PMID:25311923, PMID:4410944, PMID:6235211, PMID:6235212 Sources: DOI:10.1007/978-3-642-00286-1_2 Note: Note that this term represents protoperithecium formation across homothallic and heterothallic species that do not have the same mechanism.